{
  "gene_symbol": "GATB",
  "term_label": "mitochondrial translation",
  "term_id": "GO:0032543",
  "gene_name": "Glutamyl-tRNA(Gln) amidotransferase subunit B, mitochondrial",
  "gene": "UniProtKB:O75879"
}